{
  "gene": "UniProtKB:Q7Z7M8",
  "term_label": "Golgi membrane",
  "gene_symbol": "B3GNT8",
  "term_id": "GO:0000139",
  "gene_name": "UDP-GlcNAc:betaGal beta-1,3-N-acetylglucosaminyltransferase 8"
}